release of sequestered calcium ion into presynaptic cytosol [GO:0099585] (biological process) Relationships: is a type of release of sequestered calcium ion into cytosol [GO:0051209]; is a type of establishment of localization in cell [GO:0051649]; BFO_0000066 presynapse [GO:0098793] Definition: The process in which calcium ions sequestered in the endoplasmic reticulum, Golgi apparatus or mitochondria are released into the presynaptic cytosol. Sources: GOC:dos